{
  "gene": "UniProtKB:Q9P203",
  "term_label": "Unknown molecular function",
  "term_id": "UNKNOWN:0001",
  "gene_symbol": "BTBD7",
  "gene_name": "BTB_POZ domain-containing protein 7"
}